{
  "term_id": "GO:0005739",
  "term_label": "mitochondrion",
  "gene_symbol": "CA5BP1",
  "gene": "UniProtKB:Q8WTZ4",
  "gene_name": "Putative inactive carbonic anhydrase 5B-like protein"
}